{
  "term_id": "GO:0000981",
  "gene_symbol": "ZNF300",
  "gene": "UniProtKB:Q96RE9",
  "gene_name": "Zinc finger protein 300",
  "term_label": "DNA-binding transcription factor activity, RNA polymerase II-specific"
}